{
  "gene_symbol": "ZNF438",
  "gene": "UniProtKB:Q7Z4V0",
  "term_label": "regulation of transcription by RNA polymerase II",
  "term_id": "GO:0006357",
  "gene_name": "Zinc finger protein 438"
}